{
  "gene": "UniProtKB:P0CJ71",
  "term_id": "GO:0048019",
  "gene_symbol": "MTRNR2L4",
  "term_label": "receptor antagonist activity",
  "gene_name": "Humanin-like 4"
}